{
  "term_label": "catalytic step 2 spliceosome",
  "gene": "UniProtKB:O95926",
  "gene_symbol": "SYF2",
  "term_id": "GO:0071013",
  "gene_name": "Pre-mRNA-splicing factor SYF2"
}